{
  "term_label": "immune receptor activity",
  "term_id": "GO:0140375",
  "gene": "UniProtKB:O76036",
  "gene_symbol": "NCR1",
  "gene_name": "Natural cytotoxicity triggering receptor 1"
}